negative regulation of defense response to oomycetes [GO:1902289] (biological process) Definition: Any process that stops, prevents or reduces the frequency, rate or extent of defense response to oomycetes. References: PMID:16040633 Sources: GOC:TermGenie Also known as: down regulation of defense response to oomycetes, down-regulation of defense response to oomycetes, downregulation of defense response to oomycetes, inhibition of defense response to oomycetes Relationships: is a type of negative regulation of response to biotic stimulus [GO:0002832]; is a type of negative regulation of defense response [GO:0031348]; is a type of negative regulation of response to external stimulus [GO:0032102]; is a type of regulation of defense response to oomycetes [GO:1902288]; negatively regulates defense response to oomycetes [GO:0002229]